{
  "term_id": "GO:0005007",
  "gene_symbol": "FGFR3",
  "gene": "UniProtKB:P22607",
  "gene_name": "Fibroblast growth factor receptor 3",
  "term_label": "fibroblast growth factor receptor activity"
}